2-dehydro-3-deoxy-D-gluconic acid biosynthetic process [GO:1901274] (biological process) Sources: GOC:TermGenie, GOC:yaf, UniPathway:UPA00856 Definition: The chemical reactions and pathways resulting in the formation of 2-dehydro-3-deoxy-D-gluconic acid. Relationships: is a type of GO:0046364; is a type of GO:0072330 Also known as: 2-dehydro-3-deoxy-D-gluconic acid anabolism, 2-dehydro-3-deoxy-D-gluconic acid biosynthesis, 2-dehydro-3-deoxy-D-gluconic acid formation, 2-dehydro-3-deoxy-D-gluconic acid synthesis